protein modification by small protein conjugation or removal [GO:0070647] (BP) Regulation: regulated by regulation of protein modification by small protein conjugation or removal [GO:1903320]; negatively regulated by negative regulation of protein modification by small protein conjugation or removal [GO:1903321]; positively regulated by positive regulation of protein modification by small protein conjugation or removal [GO:1903322] Definition: A protein modification process in which one or more groups of a small protein, such as ubiquitin or a ubiquitin-like protein, are covalently attached to or removed from a target protein. Relationships: is a type of post-translational protein modification [GO:0043687] Subtypes: protein modification by small protein conjugation [GO:0032446], protein modification by small protein removal [GO:0070646] Sources: GOC:mah